hippocampal mossy fiber [GO:0097457] (cellular component) Relationships: is a type of axon [GO:0030424] Subtypes: GO:0044302 References: PMID:17765709, PMID:20554881, PMID:24336151 Sources: NIF_Subcellular:nlx_subcell_100312 Definition: An axon of a hippocampal granule cell, including dentate gyrus granule cell and CA3 granule cell, characterized by expansions (mossy fiber expansions) giving the fibers a mossy appearance. These unmyelinated axons were first described by Ramon y Cajal.